D-arabinose catabolic process [GO:0019571] (biological process) Also known as: D-arabinose breakdown, D-arabinose catabolism, D-arabinose degradation Subtypes: GO:0019573 Relationships: is a type of arabinose catabolic process [GO:0019568] Sources: GOC:jsg, GOC:mah Definition: The chemical reactions and pathways resulting in the breakdown of D-arabinose, the D-enantiomer of arabino-pentose.